{
  "gene_name": "Nuclear receptor subfamily 4 group A member 2",
  "gene": "UniProtKB:P43354",
  "gene_symbol": "NR4A2",
  "term_id": "GO:0035259",
  "term_label": "nuclear glucocorticoid receptor binding"
}